{
  "term_id": "GO:0005737",
  "term_label": "cytoplasm",
  "gene": "UniProtKB:O43795",
  "gene_name": "Unconventional myosin-Ib",
  "gene_symbol": "MYO1B"
}